{
  "term_label": "plasma membrane",
  "gene_symbol": "A0A1W2PQF6",
  "term_id": "GO:0005886",
  "gene": "UniProtKB:A0A1W2PQF6",
  "gene_name": "Immunoglobulin subtype domain-containing protein"
}